{
  "gene_symbol": "TES",
  "term_label": "Unknown cellular component",
  "term_id": "UNKNOWN:0003",
  "gene_name": "Testin",
  "gene": "UniProtKB:Q9UGI8"
}